{
  "term_label": "plasma membrane",
  "gene_symbol": "OR10G9",
  "gene_name": "Olfactory receptor 10G9",
  "term_id": "GO:0005886",
  "gene": "UniProtKB:Q8NGN4"
}